globose nucleus development [GO:0021736] (biological process) Definition: The process whose specific outcome is the progression of the globose nucleus over time, from its formation to the mature structure. Sources: GOC:cls, GOC:curators, GOC:dgh, GOC:dph, GOC:jid Relationships: is a type of neural nucleus development [GO:0048857]; is part of cerebellum development [GO:0021549]